{
  "gene_symbol": "EFNA3",
  "term_id": "GO:0048013",
  "gene_name": "Ephrin-A3",
  "term_label": "ephrin receptor signaling pathway",
  "gene": "UniProtKB:P52797"
}